{
  "term_label": "beta-1 adrenergic receptor binding",
  "gene_symbol": "MAGI2",
  "term_id": "GO:0031697",
  "gene": "UniProtKB:Q86UL8",
  "gene_name": "Membrane-associated guanylate kinase, WW and PDZ domain-containing protein 2"
}